{
  "gene": "UniProtKB:Q9UP95",
  "gene_name": "Solute carrier family 12 member 4",
  "gene_symbol": "SLC12A4",
  "term_id": "GO:0015379",
  "term_label": "potassium:chloride symporter activity"
}